negative regulation of store-operated calcium channel activity [GO:1901340] (biological process) Definition: Any process that stops, prevents or reduces the frequency, rate or extent of store-operated calcium channel activity. Relationships: is a type of negative regulation of calcium ion transmembrane transporter activity [GO:1901020]; is_a GO:1901339; negatively regulates store-operated calcium channel activity [GO:0015279] Also known as: down regulation of store-operated calcium channel activity, down-regulation of store-operated calcium channel activity, downregulation of store-operated calcium channel activity, inhibition of store-operated calcium channel activity Sources: GOC:TermGenie